{
  "gene": "UniProtKB:P60410",
  "gene_name": "Keratin-associated protein 10-8",
  "term_id": "UNKNOWN:0001",
  "term_label": "Unknown molecular function",
  "gene_symbol": "KRTAP10-8"
}